{
  "gene_symbol": "FPR2",
  "term_id": "GO:0005886",
  "gene": "UniProtKB:P25090",
  "gene_name": "N-formyl peptide receptor 2",
  "term_label": "plasma membrane"
}